digalactosyldiacylglycerol synthase activity [GO:0046481] (molecular function) Also known as: DGDG synthase activity, UDP-galactose:MGDG galactosyltransferase activity, DGD1, DGD2, UDP-galactose-dependent DGDG synthase activity, UDP-galactose-dependent digalactosyldiacylglycerol synthase activity, UDP-galactose:3-(beta-D-galactosyl)-1,2-diacyl-sn-glycerol 6-alpha-galactosyltransferase activity Sources: EC:2.4.1.241, RHEA:10520 Definition: Catalysis of the reaction: 1,2-diacyl-3-beta-D-galactosyl-sn-glycerol + UDP-D-galactose = 3-[alpha-D-galactosyl-(1->6)-beta-D-galactosyl]-1,2-diacyl-sn-glycerol + H+ + UDP. Relationships: is a type of UDP-galactosyltransferase activity [GO:0035250]